regulation of cytoplasmic translational termination [GO:1990580] (biological process) Definition: Any process that modulates the frequency, rate or extent of cytoplasmic translational termination. References: PMID:11570975 Relationships: is a type of GO:0006449; is a type of regulation of cytoplasmic translation [GO:2000765]; regulates cytoplasmic translational termination [GO:0002184]